auxin efflux transmembrane transporter activity [GO:0010329] (molecular function) References: PMID:16839804 Definition: Enables the transfer of auxin, from one side of a membrane to the other, out of a cell. Relationships: is a type of auxin transmembrane transporter activity [GO:0080161]; is part of GO:0010315 Also known as: auxin efflux carrier, auxin efflux facilitator